plantlet formation on parent plant [GO:0048624] (BP) Also known as: vegetative vivipary, vivipary Relationships: is a type of GO:0003006; is a type of GO:0019954; is_a multi-multicellular organism process [GO:0044706]; is a type of meristem development [GO:0048507]; is a type of multicellular organismal reproductive process [GO:0048609] Definition: The process in which a new plantlet develops from a meristem on the plant body. As part of this process, when the plantlet is large enough to live independently, the physical connection between the new plantlet and the main plant is severed. Sources: GOC:go_curators